regulation of [4Fe-4S] cluster assembly [GO:1900491] (biological process) Definition: Any process that modulates the frequency, rate or extent of [4Fe-4S] cluster assembly. Also known as: regulation of 4Fe-4S cluster assembly, regulation of [4Fe-4S] cluster biosynthetic process Relationships: is a type of GO:1903329; regulates [4Fe-4S] cluster assembly [GO:0044572] Sources: GOC:TermGenie, GOC:mengo_curators, GOC:pr Subtypes: negative regulation of [4Fe-4S] cluster assembly [GO:1900492], positive regulation of [4Fe-4S] cluster assembly [GO:1900493]